{
  "term_id": "UNKNOWN:0003",
  "term_label": "Unknown cellular component",
  "gene_name": "Uncharacterized protein C3orf62",
  "gene_symbol": "C3orf62",
  "gene": "UniProtKB:Q6ZUJ4"
}